negative regulation of triglyceride catabolic process [GO:0010897] (biological process) Also known as: negative regulation of triacylglycerol catabolic process Definition: Any process that decreases the frequency, rate, or extent of the chemical reactions and pathways resulting in the breakdown of triglyceride. Sources: GOC:rn, GOC:tb Relationships: is a type of GO:0010896; is a type of negative regulation of lipid catabolic process [GO:0050995]; is a type of negative regulation of triglyceride metabolic process [GO:0090209]; negatively regulates triglyceride catabolic process [GO:0019433]